{
  "gene_symbol": "SLC38A3",
  "gene_name": "Sodium-coupled neutral amino acid transporter 3",
  "gene": "UniProtKB:Q99624",
  "term_label": "plasma membrane",
  "term_id": "GO:0005886"
}